{
  "gene_name": "Transmembrane protein 50B",
  "term_id": "UNKNOWN:0003",
  "gene_symbol": "TMEM50B",
  "gene": "UniProtKB:P56557",
  "term_label": "Unknown cellular component"
}